non-motile cilium membrane [GO:0098804] (cellular component) Also known as: nonmotile primary cilium membrane Sources: GOC:cilia, GOC:dos Definition: The portion of the plasma membrane surrounding a non-motile cilium. Relationships: is_a ciliary membrane [GO:0060170]; is part of non-motile cilium [GO:0097730]